cysteine-tRNA ligase activity [GO:0004817] (MF) Also known as: cysteinyl-tRNA synthetase activity, L-cysteine:tRNACys ligase (AMP-forming), cysteine translase activity, cysteinyl-transfer ribonucleate synthetase activity, cysteinyl-transferRNA synthetase activity Relationships: is a type of aminoacyl-tRNA ligase activity [GO:0004812] Definition: Catalysis of the reaction: ATP + L-cysteine + tRNA(Cys) = AMP + diphosphate + L-cysteinyl-tRNA(Cys). Sources: EC:6.1.1.16